{
  "gene_symbol": "PURG",
  "term_label": "nucleus",
  "term_id": "GO:0005634",
  "gene": "UniProtKB:Q9UJV8",
  "gene_name": "Purine-rich element-binding protein gamma"
}